{
  "gene_symbol": "CD36",
  "gene": "UniProtKB:P16671",
  "term_label": "long-chain fatty acid import into cell",
  "term_id": "GO:0044539",
  "gene_name": "Platelet glycoprotein 4"
}